{
  "term_label": "nuclear localization sequence binding",
  "gene_symbol": "KPNA1",
  "term_id": "GO:0008139",
  "gene": "UniProtKB:P52294",
  "gene_name": "Importin subunit alpha-5"
}